{
  "gene_name": "Lutropin subunit beta",
  "term_label": "hormone activity",
  "term_id": "GO:0005179",
  "gene": "UniProtKB:P01229",
  "gene_symbol": "LHB"
}